{
  "term_id": "UNKNOWN:0001",
  "term_label": "Unknown molecular function",
  "gene": "UniProtKB:Q5HYR2",
  "gene_name": "Doublesex- and mab-3-related transcription factor C1",
  "gene_symbol": "DMRTC1"
}